{
  "term_id": "GO:0003682",
  "gene_name": "Chromodomain-helicase-DNA-binding protein 2",
  "gene": "UniProtKB:O14647",
  "term_label": "chromatin binding",
  "gene_symbol": "CHD2"
}